negative regulation of spore encystment on host [GO:0075217] (biological process) Relationships: is a type of negative regulation of cell development [GO:0010721]; is a type of modulation of spore encystment on host [GO:0075215]; RO_0002212 spore encystment [GO:0075214] Subtypes: negative regulation of zoospore encystment on host [GO:0075221] Definition: Any process that stops, prevents, or reduces the frequency, rate or extent of spore encystment on host. The host is defined as the larger of the organisms involved in a symbiotic interaction. Sources: GOC:pamgo_curators